{
  "gene": "UniProtKB:Q9P2N5",
  "term_id": "GO:0003723",
  "gene_name": "RNA-binding protein 27",
  "term_label": "RNA binding",
  "gene_symbol": "RBM27"
}